{
  "gene_name": "Trophoblast glycoprotein-like",
  "gene": "UniProtKB:P0DKB5",
  "gene_symbol": "TPBGL",
  "term_label": "negative regulation of canonical Wnt signaling pathway",
  "term_id": "GO:0090090"
}